regulation of mitotic cytokinesis, division site positioning [GO:1902472] (biological process) Relationships: is a type of regulation of mitotic cytokinetic process [GO:1903436]; is a type of regulation of cytokinesis, site selection [GO:2000073]; regulates mitotic cytokinesis, division site positioning [GO:1902408] Subtypes: positive regulation of mitotic cytokinesis, division site positioning [GO:1903617] References: PMID:9852154 Also known as: regulation of mitotic cytokinesis, site selection Definition: Any process that modulates the frequency, rate or extent of mitotic cytokinesis, division site positioning.